{
  "gene_symbol": "STK17B",
  "gene_name": "Serine_threonine-protein kinase 17B",
  "term_id": "GO:0043065",
  "term_label": "positive regulation of apoptotic process",
  "gene": "UniProtKB:O94768"
}